 [description]